{
  "term_id": "GO:0001965",
  "term_label": "G-protein alpha-subunit binding",
  "gene_name": "Adhesion G-protein coupled receptor V1",
  "gene": "UniProtKB:Q8WXG9",
  "gene_symbol": "ADGRV1"
}